{
  "gene": "UniProtKB:Q08117",
  "gene_name": "TLE family member 5",
  "gene_symbol": "TLE5",
  "term_label": "Unknown molecular function",
  "term_id": "UNKNOWN:0001"
}